{
  "term_id": "GO:0005886",
  "gene_symbol": "ADGRL2",
  "gene": "UniProtKB:O95490",
  "gene_name": "Adhesion G protein-coupled receptor L2",
  "term_label": "plasma membrane"
}